histone H3K27 monomethyltransferase activity [GO:0140953] (molecular function) Sources: RHEA:60296 Relationships: is a type of histone H3K27 methyltransferase activity [GO:0046976] Note: Comment: Note that the residue position corresponds to the canonical human H3 histone (UniProtKB:P84243); this residue is conserved across all eukaryotes. Residue 1 is the first residue following removal of the initiating Methionine (Met). Note that each histone is encoded by multiple genes, and sequences may vary across different genes within an organism. Definition: Catalysis of the reaction: L-lysyl27-[histone H3] + S-adenosyl-L-methionine = H+ + N6-methyl-L-lysyl27-[histone H3] + S-adenosyl-L-homocysteine. This reaction is the addition of a single methyl group to the unmethylated lysine residue at position 27 of histone H3, producing histone H3K27me. Also known as: histone H3-K27 methylation, histone H3K27 methylation, histone H3-K27 monomethylase activity, histone H3K27 monomethylase activity, histone lysine N-monomethyltransferase activity (H3-K27 specific)